{
  "term_id": "GO:0030258",
  "gene_name": "Ghrelin O-acyltransferase",
  "term_label": "lipid modification",
  "gene_symbol": "MBOAT4",
  "gene": "UniProtKB:Q96T53"
}